{
  "gene_name": "Neural cell adhesion molecule L1-like protein",
  "term_label": "Unknown molecular function",
  "term_id": "UNKNOWN:0001",
  "gene": "UniProtKB:O00533",
  "gene_symbol": "CHL1"
}